{
  "term_label": "Unknown molecular function",
  "term_id": "UNKNOWN:0001",
  "gene_symbol": "ASB17",
  "gene_name": "Ankyrin repeat and SOCS box protein 17",
  "gene": "UniProtKB:Q8WXJ9"
}